{
  "gene_symbol": "CLMP",
  "gene": "UniProtKB:Q9H6B4",
  "gene_name": "CXADR-like membrane protein",
  "term_label": "Unknown cellular component",
  "term_id": "UNKNOWN:0003"
}